{
  "gene_symbol": "DMXL1",
  "term_id": "GO:0007035",
  "gene": "UniProtKB:Q9Y485",
  "term_label": "vacuolar acidification",
  "gene_name": "DmX-like protein 1"
}